{
  "gene_name": "Diphosphomevalonate decarboxylase",
  "term_id": "GO:0005829",
  "term_label": "cytosol",
  "gene": "UniProtKB:P53602",
  "gene_symbol": "MVD"
}